regulation of B cell mediated immunity [GO:0002712] (biological process) Relationships: is a type of regulation of lymphocyte mediated immunity [GO:0002706]; is a type of regulation of adaptive immune response based on somatic recombination of immune receptors built from immunoglobulin superfamily domains [GO:0002822]; regulates B cell mediated immunity [GO:0019724] Also known as: regulation of B lymphocyte mediated immunity, regulation of B-cell mediated immunity, regulation of B-lymphocyte mediated immunity Definition: Any process that modulates the frequency, rate, or extent of B cell mediated immunity. Sources: GOC:add Subtypes: GO:0002622, negative regulation of B cell mediated immunity [GO:0002713], positive regulation of B cell mediated immunity [GO:0002714], GO:0002721, GO:0002889, regulation of peripheral B cell deletion [GO:0002908], regulation of peripheral B cell anergy [GO:0002917]